negative regulation of peptidyl-threonine phosphorylation [GO:0010801] (biological process) Sources: GOC:dph, GOC:tb Relationships: is_a negative regulation of protein phosphorylation [GO:0001933]; is a type of regulation of peptidyl-threonine phosphorylation [GO:0010799]; negatively regulates peptidyl-threonine phosphorylation [GO:0018107] Definition: Any process that decreases the frequency, rate or extent of peptidyl-threonine phosphorylation. Peptidyl-threonine phosphorylation is the phosphorylation of peptidyl-threonine to form peptidyl-O-phospho-L-threonine.